{
  "gene_name": "Major facilitator superfamily domain-containing 14C pseudogene",
  "gene_symbol": "MFSD14CP",
  "gene": "UniProtKB:Q5VZR4",
  "term_label": "Unknown cellular component",
  "term_id": "UNKNOWN:0003"
}